nuclear polyadenylation-dependent snoRNA catabolic process [GO:0071036] (biological process) Definition: The chemical reactions and pathways occurring in the nucleus and resulting in the breakdown of a small nucleolar RNA (snoRNA) molecule, initiated by the enzymatic addition of a sequence of adenylyl residues (polyadenylation) at the 3' end the target snoRNA. References: PMID:15935758 Sources: GOC:dgf, GOC:krc Also known as: nuclear poly(A)-dependent snoRNA catabolic process Relationships: is a type of sno(s)RNA catabolic process [GO:0016077]; is a type of nuclear RNA surveillance [GO:0071027]; has part poly(A)-dependent snoRNA 3'-end processing [GO:0071051]